{
  "gene_symbol": "LRRC7",
  "term_label": "positive regulation of neuron projection development",
  "gene": "UniProtKB:Q96NW7",
  "gene_name": "Leucine-rich repeat-containing protein 7",
  "term_id": "GO:0010976"
}